{
  "gene_name": "Magnesium transporter MRS2 homolog, mitochondrial",
  "term_label": "mitochondrial inner membrane",
  "gene": "UniProtKB:Q9HD23",
  "gene_symbol": "MRS2",
  "term_id": "GO:0005743"
}